endosome lysis involved in viral entry into host cell [GO:0075514] (biological process) Definition: Viral-induced lysis of the endosome involved in uptake of a virus into a host cell. Occurs after internalization of the virus through the endosomal pathway, and results in release of the viral contents from the endosome into the host cell cytoplasm. Sources: GOC:bf, GOC:jl Also known as: viral entry into host cell via caveolae-mediated endocytosis followed by endosome lysis Relationships: is a type of lysis of host organelle involved in viral entry into host cell [GO:0039664]